{
  "gene_symbol": "TP53I11",
  "term_label": "Unknown molecular function",
  "gene": "UniProtKB:O14683",
  "term_id": "UNKNOWN:0001",
  "gene_name": "Tumor protein p53-inducible protein 11"
}